{
  "term_label": "positive regulation of transcription by RNA polymerase II",
  "term_id": "GO:0045944",
  "gene_symbol": "RXRG",
  "gene": "UniProtKB:P48443",
  "gene_name": "Retinoic acid receptor RXR-gamma"
}